{
  "gene_name": "Putative CENPB DNA-binding domain-containing protein 1",
  "gene_symbol": "CENPBD1P",
  "gene": "UniProtKB:B2RD01",
  "term_id": "UNKNOWN:0002",
  "term_label": "Unknown biological process"
}